specification of segmental identity, antennal segment [GO:0007383] (biological process) Definition: The specification of the characteristic structures of the antennal segment following establishment of segment boundaries. Identity is considered to be the aggregate of characteristics by which a structure is recognized. Sources: ISBN:0878932437 Note: See also the fly_anatomy.ontology term 'antennal segment ; FBbt:00000009'. Relationships: is a type of specification of segmental identity, head [GO:0007380]; is part of GO:0035288